{
  "gene_name": "Mediator of RNA polymerase II transcription subunit 6",
  "gene_symbol": "MED6",
  "gene": "UniProtKB:O75586",
  "term_id": "GO:0016592",
  "term_label": "mediator complex"
}